regulation of microglial cell activation [GO:1903978] (biological process) Definition: Any process that modulates the frequency, rate or extent of microglial cell activation. References: PMID:19100238 Sources: GOC:BHF, GOC:TermGenie, GOC:nc, GO_REF:0000058 Relationships: is a type of regulation of macrophage activation [GO:0043030]; is a type of regulation of neuroinflammatory response [GO:0150077]; regulates microglial cell activation [GO:0001774] Subtypes: negative regulation of microglial cell activation [GO:1903979], positive regulation of microglial cell activation [GO:1903980]